{
  "term_id": "GO:0035269",
  "gene_name": "Xylosyl- and glucuronyltransferase LARGE1",
  "term_label": "protein O-linked glycosylation via mannose",
  "gene_symbol": "LARGE1",
  "gene": "UniProtKB:O95461"
}